{
  "term_label": "extracellular space",
  "gene": "UniProtKB:P30511",
  "gene_symbol": "HLA-F",
  "term_id": "GO:0005615",
  "gene_name": "HLA class I histocompatibility antigen, alpha chain F"
}